{
  "term_label": "intracellular signal transduction",
  "gene_symbol": "MAPK7",
  "term_id": "GO:0035556",
  "gene": "UniProtKB:Q13164",
  "gene_name": "Mitogen-activated protein kinase 7"
}